blastocyst formation [GO:0001825] (biological process) Sources: GOC:dph, ISBN:0124020607, ISBN:0198542771 Note: See also the Anatomical Dictionary for Mouse Development ontology term 'TS3, compacted morula ; EMAP:9'. Also known as: blastula formation Relationships: is a type of GO:0048646; is part of blastocyst development [GO:0001824] Definition: The initial formation of a blastocyst from a solid ball of cells known as a morula.